{
  "gene_name": "Beta-crystallin B3",
  "term_id": "GO:0007601",
  "gene_symbol": "CRYBB3",
  "term_label": "visual perception",
  "gene": "UniProtKB:P26998"
}